{
  "term_label": "mitochondrion",
  "gene": "UniProtKB:Q86WU2",
  "term_id": "GO:0005739",
  "gene_name": "Probable D-lactate dehydrogenase, mitochondrial",
  "gene_symbol": "LDHD"
}